{
  "term_id": "GO:0043020",
  "gene_name": "Cytochrome b-245 heavy chain",
  "term_label": "NADPH oxidase complex",
  "gene": "UniProtKB:P04839",
  "gene_symbol": "CYBB"
}